{
  "term_label": "neuron differentiation",
  "gene_symbol": "INSM1",
  "gene": "UniProtKB:Q01101",
  "term_id": "GO:0030182",
  "gene_name": "Insulinoma-associated protein 1"
}